{
  "gene_symbol": "SEPTIN6",
  "term_label": "cell division site",
  "gene": "UniProtKB:Q14141",
  "term_id": "GO:0032153",
  "gene_name": "Septin-6"
}